positive regulation of protein localization to prospore membrane [GO:2001232] (biological process) Relationships: is a type of positive regulation of protein localization to plasma membrane [GO:1903078]; is a type of regulation of protein localization to prospore membrane [GO:2001231]; positively regulates protein localization to prospore membrane [GO:1902657] Definition: Any process that activates or increases the frequency, rate or extent of protein localization to prospore membrane. Sources: GOC:mah Also known as: positive regulation of protein localisation to prospore membrane, positive regulation of protein targeting to FSM, positive regulation of protein targeting to ascospore-type prospore membrane, positive regulation of protein targeting to forespore membrane, positive regulation of protein targeting to prospore membrane, positive regulation of protein-prospore membrane targeting